{
  "term_label": "nucleus",
  "gene": "UniProtKB:Q96BV0",
  "gene_symbol": "ZNF775",
  "term_id": "GO:0005634",
  "gene_name": "Zinc finger protein 775"
}